{
  "gene_symbol": "PIK3CA",
  "gene_name": "Phosphatidylinositol 4,5-bisphosphate 3-kinase catalytic subunit alpha isoform",
  "term_label": "phosphatidylinositol 3-kinase complex, class IB",
  "gene": "UniProtKB:P42336",
  "term_id": "GO:0005944"
}